{
  "term_id": "GO:0046540",
  "term_label": "U4/U6 x U5 tri-snRNP complex",
  "gene": "UniProtKB:P14678",
  "gene_symbol": "SNRPB",
  "gene_name": "Small nuclear ribonucleoprotein-associated proteins B and B'"
}